extracellular matrix constituent conferring elasticity [GO:0030023] (MF) Definition: A component of the extracellular matrix that enables the matrix to recoil after transient stretching. Also known as: core extracellular matrix, core matrisome, elastin Note: Extracellular matrix elastin proteins may be annotated to this term. PMID:27009176, PMID:24443019 Sources: GOC:mah, ISBN:0815316194 Relationships: is a type of extracellular matrix structural constituent [GO:0005201]; is a type of GO:0097493